{
  "term_label": "mRNA splicing, via spliceosome",
  "term_id": "GO:0000398",
  "gene_symbol": "RBM6",
  "gene": "UniProtKB:P78332",
  "gene_name": "RNA-binding protein 6"
}